{
  "term_id": "GO:0048020",
  "gene_symbol": "CCL23",
  "gene": "UniProtKB:P55773",
  "term_label": "CCR chemokine receptor binding",
  "gene_name": "C-C motif chemokine 23"
}